{
  "term_label": "cytosol",
  "gene": "UniProtKB:Q9H0X9",
  "term_id": "GO:0005829",
  "gene_name": "Oxysterol-binding protein-related protein 5",
  "gene_symbol": "OSBPL5"
}